{
  "term_id": "UNKNOWN:0002",
  "gene_symbol": "UGT2A1",
  "gene": "UniProtKB:P0DTE4",
  "term_label": "Unknown biological process",
  "gene_name": "UDP-glucuronosyltransferase 2A1"
}